positive regulation of skeletal muscle cell differentiation [GO:2001016] (biological process) Subtypes: positive regulation of skeletal muscle satellite cell differentiation [GO:1902726], GO:1902811 Sources: GOC:obol Relationships: is a type of GO:0045597; is a type of regulation of skeletal muscle cell differentiation [GO:2001014]; positively regulates GO:0035914 Definition: Any process that activates or increases the frequency, rate or extent of skeletal muscle cell differentiation.